quercetin 3'-O-glucosyltransferase activity [GO:0080045] (molecular function) References: PMID:15352060 Relationships: is a type of UDP-glucosyltransferase activity [GO:0035251] Definition: Catalysis of the transfer of a glucosyl group from UDP-glucose to the 3'-hydroxy group of a quercetin molecule.